{
  "gene_name": "HAUS augmin-like complex subunit 8",
  "term_label": "microtubule binding",
  "gene_symbol": "HAUS8",
  "term_id": "GO:0008017",
  "gene": "UniProtKB:Q9BT25"
}